symbiont-mediated suppression of host TRAF-mediated signal transduction [GO:0039527] (biological process) Definition: A process in which a symbiont interferes with, inhibits or disrupts a TRAF-mediated signal transduction pathway in the host organism. The host is defined as the larger of the organisms involved in a symbiotic interaction. References: PMID:20335533, PMID:27387501, PMID:28522607, PMID:31311877, PMID:33372174 Sources: GOC:bf, GOC:sp Also known as: negative regulation by virus of host TRAF-mediated signal transduction, inhibition of host TRAF-mediated signal transduction by virus, suppression by virus of host TRAF activity, suppression by virus of host TRAF-mediated signal transduction, suppression by virus of host tumor necrosis factor receptor-associated factor signaling, disruption by virus of host TRAF-mediated signal transduction, inhibition of host TRAFs by virus Relationships: is a type of GO:0052029